{
  "term_label": "P granule",
  "gene_symbol": "SNRPG",
  "gene_name": "Small nuclear ribonucleoprotein G",
  "term_id": "GO:0043186",
  "gene": "UniProtKB:P62308"
}